{
  "term_label": "cytoplasm",
  "gene": "UniProtKB:Q86VS8",
  "term_id": "GO:0005737",
  "gene_name": "Protein Hook homolog 3",
  "gene_symbol": "HOOK3"
}